{
  "gene_symbol": "PYM1",
  "term_id": "GO:0005737",
  "gene": "UniProtKB:Q9BRP8",
  "term_label": "cytoplasm",
  "gene_name": "Partner of Y14 and mago"
}